{
  "term_id": "UNKNOWN:0002",
  "gene": "UniProtKB:Q9NP74",
  "gene_name": "Palmdelphin",
  "gene_symbol": "PALMD",
  "term_label": "Unknown biological process"
}